{
  "gene_symbol": "INHBC",
  "term_label": "cytokine activity",
  "gene": "UniProtKB:P55103",
  "gene_name": "Inhibin beta C chain",
  "term_id": "GO:0005125"
}